{
  "gene_symbol": "NAPB",
  "gene_name": "Beta-soluble NSF attachment protein",
  "term_label": "SNARE complex disassembly",
  "term_id": "GO:0035494",
  "gene": "UniProtKB:Q9H115"
}